{
  "gene": "UniProtKB:P20132",
  "term_id": "GO:0004794",
  "gene_symbol": "SDS",
  "gene_name": "L-serine dehydratase_L-threonine deaminase",
  "term_label": "threonine deaminase activity"
}